carbohydrate transmembrane transporter activity [GO:0015144] (molecular function) Definition: Enables the transfer of carbohydrate from one side of a membrane to the other. Subtypes: carbohydrate:monoatomic cation symporter activity [GO:0005402], GO:0008982, oligosaccharide transmembrane transporter activity [GO:0015157], polysaccharide transmembrane transporter activity [GO:0015159], arabitol transmembrane transporter activity [GO:0015167], glycerol transmembrane transporter activity [GO:0015168], L-idonate transmembrane transporter activity [GO:0015568], GO:0015575, sorbitol transmembrane transporter activity [GO:0015576], galactitol transmembrane transporter activity [GO:0015577], D-glucarate transmembrane transporter activity [GO:0042878], D-galactonate transmembrane transporter activity [GO:0042881], ABC-type carbohydrate transporter activity [GO:0043211], sugar transmembrane transporter activity [GO:0051119], GO:0051474, mannosylglycerate transmembrane transporter activity [GO:0051477], GO:0090563, glycerate transmembrane transporter activity [GO:1901974] Relationships: is a type of GO:0022857; is part of carbohydrate transmembrane transport [GO:0034219] Sources: GOC:jl, GOC:mtg_transport, ISBN:0815340729 Also known as: sugar transporter, carbohydrate transporter activity